{
  "term_label": "L-tyrosine biosynthetic process",
  "gene": "UniProtKB:P00439",
  "term_id": "GO:0006571",
  "gene_name": "Phenylalanine-4-hydroxylase",
  "gene_symbol": "PAH"
}